{
  "gene_symbol": "A0A8I5QJS6",
  "term_label": "Unknown cellular component",
  "gene_name": "Uncharacterized protein",
  "term_id": "UNKNOWN:0003",
  "gene": "UniProtKB:A0A8I5QJS6"
}